thyroxine 5-deiodinase activity [GO:0033798] (MF) Sources: RHEA:18897 Relationships: is a type of oxidoreductase activity, acting on X-H and Y-H to form an X-Y bond [GO:0046992] Definition: Catalysis of the reaction: 3,3',5'-triiodo-L-thyronine + iodide + acceptor + H+ = L-thyroxine + acceptor-H2. Also known as: diiodothyronine 5'-deiodinase activity, inner ring-deiodinating pathway, type III iodothyronine deiodinase activity, acceptor:3,3',5'-triiodo-L-thyronine oxidoreductase (iodinating) activity, iodothyronine 5-deiodinase activity, iodothyronine inner ring monodeiodinase activity